regulation of macrophage cytokine production [GO:0010935] (BP) Subtypes: negative regulation of macrophage cytokine production [GO:0010936], positive regulation of macrophage cytokine production [GO:0060907] Definition: Any process that modulates the rate, frequency or extent of macrophage cytokine production. Macrophage cytokine production is the appearance of a chemokine due to biosynthesis or secretion following a cellular stimulus, resulting in an increase in its intracellular or extracellular levels. Sources: GOC:BHF, GOC:rl Relationships: is a type of GO:0002718; regulates macrophage cytokine production [GO:0010934]